{
  "term_id": "GO:0003743",
  "gene_name": "Eukaryotic translation initiation factor 3 subunit I",
  "term_label": "translation initiation factor activity",
  "gene_symbol": "EIF3I",
  "gene": "UniProtKB:Q13347"
}